L-lysine oxidase activity [GO:0050029] (molecular function) Definition: Catalysis of the reaction: H2O + L-lysine + O2 = 6-amino-2-oxohexanoate + H2O2 + NH4+. Sources: RHEA:14437 Also known as: L-lysine alpha-oxidase activity, L-lysine:oxygen 2-oxidoreductase (deaminating), L-lysyl-alpha-oxidase activity Note: Note that this term has a MetaCyc pathway reference as the pathway only has a single step. Relationships: is a type of GO:0001716